{
  "term_id": "UNKNOWN:0001",
  "gene": "UniProtKB:Q96T75",
  "gene_symbol": "DSCR8",
  "gene_name": "Down syndrome critical region protein 8",
  "term_label": "Unknown molecular function"
}